{
  "term_label": "regulation of transcription by RNA polymerase II",
  "gene": "UniProtKB:Q01851",
  "gene_symbol": "POU4F1",
  "gene_name": "POU domain, class 4, transcription factor 1",
  "term_id": "GO:0006357"
}